{
  "gene": "UniProtKB:Q9H210",
  "term_id": "GO:0050911",
  "gene_symbol": "OR2D2",
  "term_label": "detection of chemical stimulus involved in sensory perception of smell",
  "gene_name": "Olfactory receptor 2D2"
}